{
  "gene_symbol": "HK2",
  "gene_name": "Hexokinase-2",
  "term_label": "glucose 6-phosphate metabolic process",
  "gene": "UniProtKB:P52789",
  "term_id": "GO:0051156"
}